{
  "gene_name": "Propionyl-CoA carboxylase beta chain, mitochondrial",
  "gene": "UniProtKB:P05166",
  "gene_symbol": "PCCB",
  "term_label": "Unknown biological process",
  "term_id": "UNKNOWN:0002"
}